{
  "gene_name": "Golgi integral membrane protein 4",
  "gene": "UniProtKB:O00461",
  "term_id": "GO:0016020",
  "term_label": "membrane",
  "gene_symbol": "GOLIM4"
}